{
  "term_label": "DNA-binding transcription factor activity, RNA polymerase II-specific",
  "gene": "UniProtKB:P52747",
  "gene_name": "Zinc finger protein 143",
  "term_id": "GO:0000981",
  "gene_symbol": "ZNF143"
}